{
  "gene": "UniProtKB:Q9Y483",
  "term_label": "DNA binding",
  "gene_symbol": "MTF2",
  "gene_name": "Metal-response element-binding transcription factor 2",
  "term_id": "GO:0003677"
}